{
  "gene_symbol": "TLR1",
  "term_label": "lipopeptide binding",
  "term_id": "GO:0071723",
  "gene_name": "Toll-like receptor 1",
  "gene": "UniProtKB:Q15399"
}